{
  "gene_name": "Signal transducer and activator of transcription 3",
  "gene": "UniProtKB:P40763",
  "term_label": "cytoplasm",
  "term_id": "GO:0005737",
  "gene_symbol": "STAT3"
}